{
  "gene": "UniProtKB:Q8N5N4",
  "gene_symbol": "C3orf22",
  "gene_name": "Uncharacterized protein C3orf22",
  "term_id": "UNKNOWN:0003",
  "term_label": "Unknown cellular component"
}